{
  "term_id": "UNKNOWN:0003",
  "term_label": "Unknown cellular component",
  "gene": "UniProtKB:Q0VFX4",
  "gene_name": "Putative uncharacterized protein LOC100128554",
  "gene_symbol": "Q0VFX4"
}